regulation of aorta morphogenesis [GO:1903847] (biological process) Definition: Any process that modulates the frequency, rate or extent of aorta morphogenesis. Subtypes: negative regulation of aorta morphogenesis [GO:1903848], positive regulation of aorta morphogenesis [GO:1903849] Relationships: is a type of regulation of artery morphogenesis [GO:1905651]; regulates GO:0035909 References: PMID:22269326 Sources: GOC:BHF, GOC:BHF_miRNA, GOC:TermGenie, GOC:rph, GO_REF:0000058